{
  "term_id": "UNKNOWN:0003",
  "gene_name": "Transmembrane protein 270",
  "gene": "UniProtKB:Q6UE05",
  "gene_symbol": "TMEM270",
  "term_label": "Unknown cellular component"
}